sphinganine biosynthetic process [GO:0046511] (biological process) Definition: The chemical reactions and pathways resulting in the formation of sphinganine, D-erythro-2-amino-1,3-octadecanediol. Sources: GOC:ai Also known as: dihydrosphingosine biosynthesis, dihydrosphingosine biosynthetic process, sphinganine anabolism, sphinganine biosynthesis, sphinganine formation, sphinganine synthesis Relationships: is a type of sphinganine metabolic process [GO:0006667]; is a type of diol biosynthetic process [GO:0034312]; is a type of sphingoid biosynthetic process [GO:0046520]